integrin binding [GO:0005178] (molecular function) Relationships: is a type of signaling receptor binding [GO:0005102]; is a type of protein-containing complex binding [GO:0044877]; is a type of cell adhesion molecule binding [GO:0050839] Also known as: integrin ligand Sources: GOC:ceb Definition: Binding to an integrin. Subtypes: integrin binding involved in cell-matrix adhesion [GO:0098640]